vesicle tethering complex [GO:0099023] (cellular component) Subtypes: exocyst [GO:0000145], GO:0000938, Golgi transport complex [GO:0017119], TRAPP complex [GO:0030008], HOPS complex [GO:0030897], CORVET complex [GO:0033263], GO:0070939, COPII vesicles tethering complex [GO:0106103] Definition: Any protein complex that plays a role in vesicle tethering. References: PMID:27243008 Sources: GOC:dos, GOC:vw Relationships: is a type of protein-containing complex [GO:0032991]